{
  "gene_name": "Myc target protein 1",
  "gene_symbol": "MYCT1",
  "gene": "UniProtKB:Q8N699",
  "term_label": "Unknown molecular function",
  "term_id": "UNKNOWN:0001"
}